PAR polarity complex [GO:0120157] (cellular component) Definition: A protein kinase complex that is required for the establishment of a cell polarity axis during the cell division cycle. Binds directly to activated CDC42 GTPase and is required for orchestrating a cellular gradient of CDC42. In S. cerevisiae components are: BEM1, CDC24 and CLA4; from worms to vertebrates it contains a PAR6 protein, PAR3 protein and an atypical PKC. Relationships: is_a serine/threonine protein kinase complex [GO:1902554] Also known as: apical polarity complex, BEM1-CDC24-CLA4 complex, Cdc42p GEF-PAK complex, PAR3-PAR6-atypical PKC, PAR3/PAR6/aPKC, PAR6-PAR3-aPKC complex Note: "This tripartite complex named PAR6/PAR3/aPKC is conserved from worms to vertebrates" (PMID:18005931). In yeast, the components are BEM1, CDC24, and CLA4. References: PMID:11113154, PMID:18005931, PMID:22500799, PMID:28682236 Sources: GOC:lnp